{
  "gene": "UniProtKB:Q8N8A6",
  "term_id": "UNKNOWN:0001",
  "gene_name": "ATP-dependent RNA helicase DDX51",
  "gene_symbol": "DDX51",
  "term_label": "Unknown molecular function"
}